{
  "gene_symbol": "SMC4",
  "gene": "UniProtKB:Q9NTJ3",
  "term_id": "UNKNOWN:0001",
  "gene_name": "Structural maintenance of chromosomes protein 4",
  "term_label": "Unknown molecular function"
}